{
  "term_id": "UNKNOWN:0003",
  "gene_name": "Inter-alpha-trypsin inhibitor heavy chain H5",
  "gene_symbol": "ITIH5",
  "term_label": "Unknown cellular component",
  "gene": "UniProtKB:Q86UX2"
}